positive regulation of cell cycle process [GO:0090068] (BP) Relationships: is a type of GO:0010564; is a type of positive regulation of cell cycle [GO:0045787]; positively regulates cell cycle process [GO:0022402] Definition: Any process that increases the rate, frequency or extent of a cellular process that is involved in the progression of biochemical and morphological phases and events that occur in a cell during successive cell replication or nuclear replication events. Sources: GOC:dph, GOC:tb Subtypes: GO:0010571, positive regulation of mitotic spindle pole body separation [GO:0010696], positive regulation of centrosome duplication [GO:0010825], positive regulation of telomere maintenance via semi-conservative replication [GO:0032215], positive regulation of cytokinesis [GO:0032467], positive regulation of DNA endoreduplication [GO:0032877], positive regulation of meiotic nuclear division [GO:0045836], positive regulation of mitotic nuclear division [GO:0045840], positive regulation of sister chromatid cohesion [GO:0045876], positive regulation of centriole replication [GO:0046601], GO:0046604, GO:0046607, positive regulation of chromosome segregation [GO:0051984], positive regulation of G0 to G1 transition [GO:0070318], positive regulation of ascospore formation [GO:0075296], positive regulation of mitotic cell cycle spindle assembly checkpoint [GO:0090267], GO:0110028, GO:0120266, positive regulation of mitotic recombination-dependent replication fork processing [GO:0120292], positive regulation of oocyte karyosome formation [GO:0120315], positive regulation of cell cycle switching, mitotic to meiotic cell cycle [GO:0140648], GO:0140748, positive regulation of cell septum assembly [GO:1901893], positive regulation of cell cycle phase transition [GO:1901989], GO:1903127, positive regulation of meiotic DNA double-strand break formation [GO:1903343], GO:1903380, positive regulation of G1 to G0 transition [GO:1903452], GO:1904146, GO:1904291, GO:1904728, positive regulation of synaptonemal complex assembly [GO:1905088], positive regulation of meiosis I spindle assembly checkpoint [GO:1905326], positive regulation of mitotic nuclear envelope disassembly [GO:1905559], positive regulation of chromosome separation [GO:1905820], positive regulation of spindle assembly [GO:1905832]